{
  "term_id": "GO:0005721",
  "gene_symbol": "CBX1",
  "gene_name": "Chromobox protein homolog 1",
  "gene": "UniProtKB:P83916",
  "term_label": "pericentric heterochromatin"
}